{
  "term_label": "3M complex",
  "gene": "UniProtKB:O75147",
  "gene_symbol": "OBSL1",
  "term_id": "GO:1990393",
  "gene_name": "Obscurin-like protein 1"
}